glomerular endothelium development [GO:0072011] (biological process) Sources: GOC:mtg_kidney_jan10 Relationships: is a type of endothelium development [GO:0003158]; is a type of GO:0072010; is part of GO:0072012 Definition: The process whose specific outcome is the progression of the glomerular endothelium over time, from its formation to the mature structure. The glomerular endothelium is an epithelial tissue that covers the internal surfaces of the glomerulus. Subtypes: metanephric glomerular endothelium development [GO:0072264]